{
  "gene": "UniProtKB:P19224",
  "gene_name": "UDP-glucuronosyltransferase 1-6",
  "gene_symbol": "UGT1A6",
  "term_label": "sterol metabolic process",
  "term_id": "GO:0016125"
}